pollen tube tip [GO:0090404] (cellular component) Sources: GOC:tb, PO:0025195, PO:0025281 Relationships: is a type of growing cell tip [GO:0035838]; is part of pollen tube [GO:0090406] Definition: The region at growing end of the pollen tube cell, where polarized growth occurs.